{
  "term_label": "Unknown biological process",
  "term_id": "UNKNOWN:0002",
  "gene_symbol": "TRAJ42",
  "gene_name": "T cell receptor alpha joining 42",
  "gene": "UniProtKB:A0A075B6Y9"
}